melanosome lumen [GO:0034493] (cellular component) Relationships: is a type of cytoplasmic vesicle lumen [GO:0060205]; is part of GO:0042470 Definition: The volume enclosed by the melanosome membrane. Sources: GOC:rph